{
  "term_id": "GO:0000978",
  "gene_name": "Zinc finger and SCAN domain-containing protein 31",
  "gene": "UniProtKB:Q96LW9",
  "gene_symbol": "ZSCAN31",
  "term_label": "RNA polymerase II cis-regulatory region sequence-specific DNA binding"
}